{
  "term_label": "olfactory receptor activity",
  "gene_symbol": "OR5M10",
  "term_id": "GO:0004984",
  "gene": "UniProtKB:Q6IEU7",
  "gene_name": "Olfactory receptor 5M10"
}